{
  "term_id": "GO:0000177",
  "gene": "UniProtKB:Q96B26",
  "term_label": "cytoplasmic exosome (RNase complex)",
  "gene_name": "Exosome complex component RRP43",
  "gene_symbol": "EXOSC8"
}